light-activated monoatomic ion channel activity [GO:0010461] (molecular function) Relationships: is a type of monoatomic ion channel activity [GO:0005216] Definition: Enables the transmembrane transfer of a monoatomic ion by a channel that opens in response to a light stimulus. Subtypes: light-activated voltage-gated calcium channel activity [GO:0008086] Sources: GOC:dph, GOC:tb